{
  "term_label": "cytokine activity",
  "term_id": "GO:0005125",
  "gene_name": "Interferon alpha-10",
  "gene": "UniProtKB:P01566",
  "gene_symbol": "IFNA10"
}